{
  "gene": "UniProtKB:Q9Y5K6",
  "term_label": "vesicle",
  "gene_name": "CD2-associated protein",
  "term_id": "GO:0031982",
  "gene_symbol": "CD2AP"
}